positive regulation of maltose transport [GO:1902345] (biological process) References: PMID:23770568 Sources: GOC:TermGenie, GOC:dph Relationships: is_a GO:0051050; is a type of regulation of maltose transport [GO:1902343]; positively regulates maltose transport [GO:0015768] Also known as: up regulation of maltose transport, up-regulation of maltose transport, upregulation of maltose transport, activation of maltose transport Definition: Any process that activates or increases the frequency, rate or extent of maltose transport.